{
  "gene": "UniProtKB:P21754",
  "term_label": "binding of sperm to zona pellucida",
  "term_id": "GO:0007339",
  "gene_symbol": "ZP3",
  "gene_name": "Zona pellucida sperm-binding protein 3"
}